{
  "gene": "UniProtKB:Q9Y266",
  "term_label": "unfolded protein binding",
  "gene_symbol": "NUDC",
  "gene_name": "Nuclear migration protein nudC",
  "term_id": "GO:0051082"
}